{
  "gene_symbol": "NELL1",
  "term_label": "protein kinase C binding",
  "gene": "UniProtKB:Q92832",
  "gene_name": "Protein kinase C-binding protein NELL1",
  "term_id": "GO:0005080"
}